positive regulation of cytokine production [GO:0001819] (biological process) Definition: Any process that activates or increases the frequency, rate or extent of production of a cytokine. Relationships: is a type of regulation of cytokine production [GO:0001817]; is a type of positive regulation of gene expression [GO:0010628]; is a type of positive regulation of multicellular organismal process [GO:0051240]; positively regulates cytokine production [GO:0001816] Also known as: up regulation of cytokine production, up-regulation of cytokine production, upregulation of cytokine production, activation of cytokine production, positive regulation of cytokine biosynthetic process, positive regulation of cytokine secretion, stimulation of cytokine production Subtypes: positive regulation of cytokine production involved in immune response [GO:0002720], positive regulation of vascular endothelial growth factor production [GO:0010575], positive regulation of type I interferon production [GO:0032481], positive regulation of chemokine production [GO:0032722], positive regulation of connective tissue growth factor production [GO:0032723], positive regulation of granulocyte macrophage colony-stimulating factor production [GO:0032725], GO:0032726, positive regulation of type II interferon production [GO:0032729], GO:0032732, GO:0032733, positive regulation of interleukin-11 production [GO:0032734], positive regulation of interleukin-12 production [GO:0032735], positive regulation of interleukin-13 production [GO:0032736], positive regulation of interleukin-15 production [GO:0032738], positive regulation of interleukin-16 production [GO:0032739], positive regulation of interleukin-17 production [GO:0032740], positive regulation of interleukin-18 production [GO:0032741], positive regulation of interleukin-19 production [GO:0032742], positive regulation of interleukin-2 production [GO:0032743], positive regulation of interleukin-20 production [GO:0032744], positive regulation of interleukin-21 production [GO:0032745], positive regulation of interleukin-22 production [GO:0032746], positive regulation of interleukin-23 production [GO:0032747], GO:0032748, positive regulation of interleukin-25 production [GO:0032749], positive regulation of interleukin-26 production [GO:0032750], GO:0032751, GO:0032752, GO:0032753, GO:0032754, positive regulation of interleukin-6 production [GO:0032755], positive regulation of interleukin-7 production [GO:0032756], positive regulation of interleukin-8 production [GO:0032757], GO:0032758, GO:0034346, positive regulation of interleukin-35 production [GO:0070756], positive regulation of transforming growth factor beta production [GO:0071636], positive regulation of fibroblast growth factor production [GO:0090271], positive regulation of platelet-derived growth factor production [GO:0090362], positive regulation of amphiregulin production [GO:0140732], positive regulation of interleukin-33 production [GO:0150129], positive regulation of interleukin-37 production [GO:0150139], positive regulation of interleukin-34 production [GO:0150158], GO:0150191, positive regulation of cytokine production involved in inflammatory response [GO:1900017], GO:1900168, positive regulation of macrophage colony-stimulating factor production [GO:1901258], positive regulation of tumor necrosis factor superfamily cytokine production [GO:1903557], positive regulation of endothelin production [GO:1904472] Sources: GOC:add, ISBN:0781735149